RNA polymerase complex [GO:0030880] (cellular component) Definition: Any complex that possesses RNA polymerase activity; generally comprises a catalytic subunit and one or more additional subunits. Relationships: is a type of transferase complex, transferring phosphorus-containing groups [GO:0061695]; is a type of intracellular protein-containing complex [GO:0140535] Sources: GOC:mah Also known as: multisubunit RNA polymerase Subtypes: GO:0000428, GO:0031379